{
  "term_label": "phosphatidylinositol-4,5-bisphosphate 5-phosphatase activity",
  "gene_symbol": "SYNJ1",
  "term_id": "GO:0004439",
  "gene_name": "Synaptojanin-1",
  "gene": "UniProtKB:O43426"
}